oligopeptidase activity [GO:0070012] (molecular function) Definition: Catalysis of the hydrolysis of a peptide bond in an oligopeptide, i.e. a molecule containing a small number (2 to 20) of amino acid residues connected by peptide bonds. Sources: GOC:mah, ISBN:0198506732 Relationships: is a type of GO:0004175